determination of left/right asymmetry in nervous system [GO:0035545] (BP) References: PMID:17717195, PMID:19641012 Sources: GOC:kmv Definition: The establishment of the nervous system with respect to the left and right halves. Subtypes: determination of left/right asymmetry in diencephalon [GO:0035462] Relationships: is a type of determination of left/right symmetry [GO:0007368]; is part of nervous system development [GO:0007399]